{
  "term_id": "UNKNOWN:0001",
  "term_label": "Unknown molecular function",
  "gene_symbol": "TNRC18",
  "gene": "UniProtKB:O15417",
  "gene_name": "Trinucleotide repeat-containing gene 18 protein"
}